{
  "gene_name": "Protein FAM209A",
  "term_label": "Unknown biological process",
  "gene_symbol": "FAM209A",
  "gene": "UniProtKB:Q5JX71",
  "term_id": "UNKNOWN:0002"
}